{
  "term_label": "Unknown biological process",
  "term_id": "UNKNOWN:0002",
  "gene_name": "SCY1-like protein 2",
  "gene": "UniProtKB:Q6P3W7",
  "gene_symbol": "SCYL2"
}